{
  "gene": "UniProtKB:Q8TAW3",
  "term_label": "RNA polymerase II cis-regulatory region sequence-specific DNA binding",
  "term_id": "GO:0000978",
  "gene_name": "Zinc finger protein 671",
  "gene_symbol": "ZNF671"
}